{
  "gene": "UniProtKB:Q9UGP4",
  "gene_symbol": "LIMD1",
  "term_label": "transcription regulator complex",
  "gene_name": "LIM domain-containing protein 1",
  "term_id": "GO:0005667"
}